{
  "term_label": "peptide catabolic process",
  "gene_symbol": "ANPEP",
  "term_id": "GO:0043171",
  "gene": "UniProtKB:P15144",
  "gene_name": "Aminopeptidase N"
}